establishment of cell polarity involved in mesendodermal cell migration [GO:0003369] (biological process) Sources: GOC:ascb_2009, GOC:dph, GOC:tb Relationships: is a type of GO:0003379; is part of cell migration involved in mesendoderm migration [GO:0090134] Definition: The specification and formation of anisotropic intracellular organization that contributes to the self-propelled directed movement of a mesendodermal cell.